{
  "gene_symbol": "MBIP",
  "term_label": "cytosol",
  "gene": "UniProtKB:Q9NS73",
  "gene_name": "MAP3K12-binding inhibitory protein 1",
  "term_id": "GO:0005829"
}